{
  "term_id": "GO:0005634",
  "term_label": "nucleus",
  "gene_symbol": "SIRT1",
  "gene_name": "NAD-dependent protein deacetylase sirtuin-1",
  "gene": "UniProtKB:Q96EB6"
}